anterior lateral line neuromast mantle cell differentiation [GO:0048905] (biological process) Sources: ISBN:0125296509 Relationships: is a type of neuromast mantle cell differentiation [GO:0048888]; is part of anterior lateral line neuromast development [GO:0048901] Definition: The process in which a relatively unspecialized cell acquires specialized features of an anterior lateral line neuromast mantle cell. Mantle cells are non-sensory cells that surround the sensory strip, separating the neuromast from the epidermis. Mantle cells secrete the cupula in which the ciliary bundles of all of the hair cells are embedded.